{
  "gene": "UniProtKB:Q5TCY1",
  "term_id": "GO:0005634",
  "gene_name": "Tau-tubulin kinase 1",
  "term_label": "nucleus",
  "gene_symbol": "TTBK1"
}